{
  "gene_symbol": "RPS6KA4",
  "term_label": "protein serine/threonine kinase activity",
  "term_id": "GO:0004674",
  "gene_name": "Ribosomal protein S6 kinase alpha-4",
  "gene": "UniProtKB:O75676"
}